{
  "gene_name": "Desmoglein-1",
  "gene_symbol": "DSG1",
  "gene": "UniProtKB:Q02413",
  "term_id": "GO:0045295",
  "term_label": "gamma-catenin binding"
}